{
  "term_label": "Unknown molecular function",
  "term_id": "UNKNOWN:0001",
  "gene": "UniProtKB:A6NL46",
  "gene_name": "Putative UPF0607 protein ENSP00000332738",
  "gene_symbol": "A6NL46"
}